{
  "gene_symbol": "IYD",
  "term_id": "GO:0005886",
  "term_label": "plasma membrane",
  "gene": "UniProtKB:Q6PHW0",
  "gene_name": "Iodotyrosine deiodinase 1"
}